optic cup morphogenesis involved in camera-type eye development [GO:0002072] (biological process) Sources: GOC:dph, GOC:mtg_sensu, GOC:sdb_2009, GOC:tb, ISBN:0878932437 Relationships: is a type of GO:0016331; is part of GO:0060900 Definition: The invagination of the optic vesicle to form two-walled indentations, the optic cups, that will go on to form the retina. This process begins with the optic vesicle becoming a two-walled structure and its subsequent shape changes. It does not include the fate commitment of cells to become the pigmented retina and the neural retina. An example of this process is found in Mus musculus. Also known as: optic cup morphogenesis involved in camera-style eye development